{
  "gene_name": "Dynamin-like 120 kDa protein, mitochondrial",
  "gene_symbol": "OPA1",
  "gene": "UniProtKB:O60313",
  "term_label": "microtubule binding",
  "term_id": "GO:0008017"
}